{
  "gene": "UniProtKB:Q7Z7A3",
  "term_id": "GO:0002144",
  "gene_name": "Cytoplasmic tRNA 2-thiolation protein 1",
  "term_label": "cytosolic tRNA wobble base thiouridylase complex",
  "gene_symbol": "CTU1"
}